{
  "term_id": "GO:0000149",
  "gene_symbol": "SYT8",
  "gene_name": "Synaptotagmin-8",
  "gene": "UniProtKB:Q8NBV8",
  "term_label": "SNARE binding"
}